{
  "gene_symbol": "C11orf98",
  "gene_name": "Uncharacterized protein C11orf98",
  "term_label": "Unknown molecular function",
  "term_id": "UNKNOWN:0001",
  "gene": "UniProtKB:E9PRG8"
}